positive regulation of neurotransmitter secretion [GO:0001956] (biological process) Sources: GOC:hjd Definition: Any process that activates or increases the frequency, rate or extent of the regulated release of a neurotransmitter. Also known as: up regulation of neurotransmitter secretion, up-regulation of neurotransmitter secretion, upregulation of neurotransmitter secretion, activation of neurotransmitter secretion, stimulation of neurotransmitter secretion Relationships: is_a regulation of neurotransmitter secretion [GO:0046928]; is a type of GO:0050806; is a type of positive regulation of neurotransmitter transport [GO:0051590]; is a type of GO:1903532; positively regulates neurotransmitter secretion [GO:0007269] Subtypes: positive regulation of acetylcholine secretion, neurotransmission [GO:0014057], positive regulation of glutamate secretion, neurotransmission [GO:1903296], positive regulation of spontaneous neurotransmitter secretion [GO:1904050], positive regulation of substance P secretion, neurotransmission [GO:1904496], positive regulation of glycine secretion, neurotransmission [GO:1904626], positive regulation of synaptic vesicle exocytosis [GO:2000302]